{
  "term_label": "nucleus",
  "gene": "UniProtKB:Q99828",
  "term_id": "GO:0005634",
  "gene_symbol": "CIB1",
  "gene_name": "Calcium and integrin-binding protein 1"
}